{
  "gene_symbol": "IGDCC4",
  "gene_name": "Immunoglobulin superfamily DCC subclass member 4",
  "term_id": "UNKNOWN:0001",
  "gene": "UniProtKB:Q8TDY8",
  "term_label": "Unknown molecular function"
}